{
  "gene": "UniProtKB:Q96AP7",
  "gene_symbol": "ESAM",
  "gene_name": "Endothelial cell-selective adhesion molecule",
  "term_label": "cell-cell adhesion mediator activity",
  "term_id": "GO:0098632"
}